{
  "gene_name": "Spermatogenesis- and oogenesis-specific basic helix-loop-helix-containing protein 1",
  "term_label": "nucleus",
  "gene": "UniProtKB:Q5JUK2",
  "gene_symbol": "SOHLH1",
  "term_id": "GO:0005634"
}